{
  "gene_symbol": "GABARAPL2",
  "gene": "UniProtKB:P60520",
  "term_id": "GO:0008429",
  "term_label": "phosphatidylethanolamine binding",
  "gene_name": "Gamma-aminobutyric acid receptor-associated protein-like 2"
}